{
  "gene_name": "Lysosome-associated membrane glycoprotein 2",
  "term_id": "GO:0061740",
  "gene": "UniProtKB:P13473",
  "term_label": "protein targeting to lysosome involved in chaperone-mediated autophagy",
  "gene_symbol": "LAMP2"
}